{
  "gene_symbol": "CWC15",
  "term_id": "GO:0071013",
  "gene_name": "Spliceosome-associated protein CWC15 homolog",
  "gene": "UniProtKB:Q9P013",
  "term_label": "catalytic step 2 spliceosome"
}